{
  "term_label": "plasma membrane",
  "term_id": "GO:0005886",
  "gene": "UniProtKB:O75558",
  "gene_symbol": "STX11",
  "gene_name": "Syntaxin-11"
}